{
  "gene": "UniProtKB:P58872",
  "term_label": "serine-type endopeptidase activity",
  "term_id": "GO:0004252",
  "gene_symbol": "RHBDL3",
  "gene_name": "Rhomboid-related protein 3"
}